{
  "term_label": "protein serine/threonine kinase activity",
  "gene_name": "Maternal embryonic leucine zipper kinase",
  "gene": "UniProtKB:Q14680",
  "gene_symbol": "MELK",
  "term_id": "GO:0004674"
}